{
  "gene_symbol": "HAVCR1",
  "term_label": "cell surface",
  "term_id": "GO:0009986",
  "gene_name": "Hepatitis A virus cellular receptor 1",
  "gene": "UniProtKB:Q96D42"
}